{
  "term_label": "protein serine/threonine kinase activator activity",
  "gene_symbol": "ETAA1",
  "term_id": "GO:0043539",
  "gene_name": "Ewing's tumor-associated antigen 1",
  "gene": "UniProtKB:Q9NY74"
}